SCF-Mdm30 ubiquitin ligase complex [GO:0097665] (cellular component) Definition: An SCF ubiquitin ligase complex in which the F-box protein is Mdm30 in S. cerevisiae. References: PMID:14747994 Sources: GOC:jd, GOC:vw Relationships: is a type of SCF ubiquitin ligase complex [GO:0019005]